{
  "gene_symbol": "SRP9",
  "term_id": "GO:0005786",
  "gene": "UniProtKB:P49458",
  "gene_name": "Signal recognition particle 9 kDa protein",
  "term_label": "signal recognition particle, endoplasmic reticulum targeting"
}